positive regulation of plasmacytoid dendritic cell cytokine production [GO:0002738] (biological process) Definition: Any process that activates or increases the frequency, rate, or extent of plasmacytoid dendritic cell cytokine production. Relationships: is a type of positive regulation of dendritic cell cytokine production [GO:0002732]; is a type of regulation of plasmacytoid dendritic cell cytokine production [GO:0002736]; positively regulates plasmacytoid dendritic cell cytokine production [GO:0002373] Also known as: up regulation of plasmacytoid dendritic cell cytokine production, up-regulation of plasmacytoid dendritic cell cytokine production, upregulation of plasmacytoid dendritic cell cytokine production, activation of plasmacytoid dendritic cell cytokine production, stimulation of plasmacytoid dendritic cell cytokine production Sources: GOC:add